{
  "gene": "UniProtKB:O75146",
  "term_label": "clathrin-coated vesicle",
  "gene_name": "Huntingtin-interacting protein 1-related protein",
  "term_id": "GO:0030136",
  "gene_symbol": "HIP1R"
}